{
  "gene": "UniProtKB:O00626",
  "gene_name": "C-C motif chemokine 22",
  "term_label": "antimicrobial humoral immune response mediated by antimicrobial peptide",
  "term_id": "GO:0061844",
  "gene_symbol": "CCL22"
}